{
  "gene_symbol": "GAREM2",
  "term_id": "UNKNOWN:0002",
  "gene_name": "GRB2-associated and regulator of MAPK protein 2",
  "term_label": "Unknown biological process",
  "gene": "UniProtKB:Q75VX8"
}